{
  "gene_symbol": "ZNF582",
  "gene": "UniProtKB:Q96NG8",
  "term_label": "regulation of transcription by RNA polymerase II",
  "gene_name": "Zinc finger protein 582",
  "term_id": "GO:0006357"
}